fibroblast growth factor receptor signaling pathway involved in neural plate anterior/posterior pattern formation [GO:0060825] (biological process) Also known as: fibroblast growth factor receptor signalling pathway involved in neural plate anterior/posterior pattern formation Subtypes: negative regulation of anterior neural cell fate commitment of the neural plate by fibroblast growth factor receptor signaling pathway [GO:0022003] Sources: GOC:dph, GOC:sdb_2009, GOC:tb Definition: The series of molecular signals generated as a consequence of a fibroblast growth factor receptor binding to one of its physiological ligands contributing to the anterior/posterior pattern of the neural plate. Regulation: regulated by regulation of fibroblast growth factor receptor signaling pathway involved in neural plate anterior/posterior pattern formation [GO:2000313]; negatively regulated by GO:2000314; positively regulated by GO:2000315 Relationships: is a type of GO:0008543; is part of neural plate anterior/posterior regionalization [GO:0021999]